L-histidine catabolic process to hydantoin-5-propionate [GO:0019560] (biological process) Relationships: is a type of L-histidine catabolic process [GO:0006548]; is a type of monocarboxylic acid metabolic process [GO:0032787] Also known as: histidine breakdown to hydantoin-5-propionate, histidine degradation to hydantoin-5-propionate Definition: The chemical reactions and pathways resulting in the breakdown of L-histidine into other compounds, including hydantoin-5-propionate. Sources: GOC:go_curators